{
  "gene": "UniProtKB:Q9Y238",
  "gene_name": "Deleted in lung and esophageal cancer protein 1",
  "term_id": "UNKNOWN:0002",
  "term_label": "Unknown biological process",
  "gene_symbol": "DLEC1"
}